{
  "gene": "UniProtKB:Q9UKY1",
  "gene_name": "Zinc fingers and homeoboxes protein 1",
  "term_id": "GO:0005634",
  "gene_symbol": "ZHX1",
  "term_label": "nucleus"
}